growth plate cartilage axis specification [GO:0003421] (biological process) Also known as: growth plate cartilage axis determination Relationships: is a type of GO:0009798; is part of GO:0003422 Sources: GOC:ascb_2009, GOC:dph, GOC:tb Definition: The establishment, maintenance and elaboration of the columnar cartilage along the axis of a long bone that contributes to bone growth.